{
  "gene_name": "Regulator of G-protein signaling 5",
  "term_id": "GO:0005096",
  "gene_symbol": "RGS5",
  "gene": "UniProtKB:O15539",
  "term_label": "GTPase activator activity"
}